diacylglycerol acyl-chain remodeling [GO:0036154] (BP) Also known as: diacylglycerol acyl-chain remodelling, diglyceride acyl-chain remodeling Relationships: is a type of acylglycerol acyl-chain remodeling [GO:0036155]; is a type of diacylglycerol metabolic process [GO:0046339] Definition: Remodeling the acyl chains of diacylglycerol, through sequential deacylation and re-acylation reactions, to generate diacylglycerol containing different types of fatty acid acyl chains. References: PMID:15364929 Sources: GOC:mw